positive regulation of alpha-beta T cell activation [GO:0046635] (BP) Definition: Any process that activates or increases the frequency, rate or extent of alpha-beta T cell activation. Sources: GOC:ai Also known as: positive regulation of alpha-beta T lymphocyte activation, positive regulation of alpha-beta T-cell activation, positive regulation of alpha-beta T-lymphocyte activation, up regulation of alpha-beta T cell activation, up-regulation of alpha-beta T cell activation, upregulation of alpha-beta T cell activation, activation of alpha-beta T cell activation, stimulation of alpha-beta T cell activation Relationships: is a type of regulation of alpha-beta T cell activation [GO:0046634]; is a type of positive regulation of T cell activation [GO:0050870]; positively regulates GO:0046631 Subtypes: GO:0046638, positive regulation of alpha-beta T cell proliferation [GO:0046641], positive regulation of NK T cell activation [GO:0051135], positive regulation of CD4-positive, alpha-beta T cell activation [GO:2000516], positive regulation of CD8-positive, alpha-beta T cell activation [GO:2001187]